{
  "term_label": "Unknown cellular component",
  "gene_name": "Protein FAM241B",
  "gene": "UniProtKB:Q96D05",
  "gene_symbol": "FAM241B",
  "term_id": "UNKNOWN:0003"
}